venom-mediated perturbation of ion channel activity [GO:0044560] (biological process) Definition: A process in which an organism alters or subverts the activity of an ion channel in another organism via the action of a venom. Subtypes: venom-mediated perturbation of calcium channel activity [GO:0044472], venom-mediated perturbation of voltage-gated sodium channel activity [GO:0044492], venom-mediated perturbation of voltage-gated potassium channel activity [GO:0044559], venom-mediated perturbation of pH-gated ion channel activity [GO:0044733] Also known as: envenomation resulting in modulation of ion channel activity in another organism, envenomation resulting in modulation of ion channel activity in other organism, envenomation resulting in regulation of ion channel activity in other organism Relationships: is a type of venom-mediated perturbation of biological process [GO:0035738] Sources: GOC:fj, GOC:jl